{
  "gene_symbol": "GRM8",
  "gene": "UniProtKB:O00222",
  "term_label": "plasma membrane",
  "gene_name": "Metabotropic glutamate receptor 8",
  "term_id": "GO:0005886"
}